{
  "term_label": "adenylate cyclase-activating G protein-coupled receptor signaling pathway",
  "term_id": "GO:0007189",
  "gene": "UniProtKB:P32245",
  "gene_name": "Melanocortin receptor 4",
  "gene_symbol": "MC4R"
}